{
  "gene_symbol": "ASNS",
  "term_id": "GO:0005829",
  "gene": "UniProtKB:P08243",
  "gene_name": "Asparagine synthetase [glutamine-hydrolyzing]",
  "term_label": "cytosol"
}